{
  "gene_symbol": "ERVK-6",
  "term_label": "Unknown biological process",
  "term_id": "UNKNOWN:0002",
  "gene": "UniProtKB:Q9BXR3",
  "gene_name": "Endogenous retrovirus group K member 6 Pol protein"
}